{
  "term_id": "GO:0000978",
  "gene_name": "Max-like protein X",
  "gene_symbol": "MLX",
  "gene": "UniProtKB:Q9UH92",
  "term_label": "RNA polymerase II cis-regulatory region sequence-specific DNA binding"
}